regulation of phospholipase C-activating G protein-coupled receptor signaling pathway [GO:1900736] (biological process) Definition: Any process that modulates the frequency, rate or extent of phospholipase C-activating G protein-coupled receptor signaling pathway. Subtypes: negative regulation of phospholipase C-activating G protein-coupled receptor signaling pathway [GO:1900737], positive regulation of phospholipase C-activating G protein-coupled receptor signaling pathway [GO:1900738] Relationships: is_a regulation of G protein-coupled receptor signaling pathway [GO:0008277]; regulates GO:0007200 Sources: GOC:BHF, GOC:TermGenie Also known as: regulation of G protein signaling, coupled to IP3 second messenger (phospholipase C activating), regulation of G protein signalling, coupled to IP3 second messenger (phospholipase C activating), regulation of G-protein coupled receptor signaling pathway coupled to IP3 second messenger, regulation of G-protein signaling, coupled to IP3 second messenger (phospholipase C activating), regulation of G-protein signalling, coupled to IP3 second messenger (phospholipase C activating), regulation of PLC-activating GPCR signaling pathway, regulation of phospholipase C-activating G-protein coupled receptor signaling pathway, regulation of phospholipase C-activating dopamine receptor signaling pathway, regulation of activation of phospholipase C activity by G-protein coupled receptor protein signaling pathway coupled to IP3 second messenger